{
  "term_label": "response to toxic substance",
  "gene": "UniProtKB:Q13867",
  "gene_name": "Bleomycin hydrolase",
  "gene_symbol": "BLMH",
  "term_id": "GO:0009636"
}